{
  "term_id": "GO:0005834",
  "gene": "UniProtKB:Q5JWF2",
  "term_label": "heterotrimeric G-protein complex",
  "gene_name": "Guanine nucleotide-binding protein G(s) subunit alpha isoforms XLas",
  "gene_symbol": "GNAS"
}